{
  "gene_name": "Type 2 DNA topoisomerase 6 subunit B-like",
  "term_id": "GO:0042138",
  "term_label": "meiotic DNA double-strand break formation",
  "gene_symbol": "TOP6BL",
  "gene": "UniProtKB:Q8N6T0"
}